{
  "gene": "UniProtKB:Q9BT17",
  "gene_name": "Mitochondrial ribosome-associated GTPase 1",
  "gene_symbol": "MTG1",
  "term_id": "GO:1902775",
  "term_label": "mitochondrial large ribosomal subunit assembly"
}